{
  "term_label": "negative regulation of amyloid precursor protein biosynthetic process",
  "gene_symbol": "ITM2B",
  "term_id": "GO:0042985",
  "gene": "UniProtKB:Q9Y287",
  "gene_name": "Integral membrane protein 2B"
}